{
  "term_id": "UNKNOWN:0001",
  "gene_name": "Leucine-rich repeat protein SHOC-2",
  "gene_symbol": "SHOC2",
  "term_label": "Unknown molecular function",
  "gene": "UniProtKB:Q9UQ13"
}